symbiont-mediated suppression of host cytoplasmic pattern recognition receptor signaling pathway via inhibition of MDA-5 activity [GO:0039554] (biological process) Relationships: is a type of symbiont-mediated suppression of cytoplasmic pattern recognition receptor signaling pathway [GO:0039537] Also known as: suppression by virus of host viral-induced cytoplasmic pattern recognition receptor signaling pathway via inhibition of host MDA-5 activity, Inhibition of host MDA5 by virus, inhibition by virus of host MDA-5 signaling, inhibition of host IFIH1/MDA5 by virus, suppression by virus of host IFIH1 signaling pathway, suppression by virus of host MDA-5 activity, suppression by virus of host MDA-5 signaling pathway, suppression by virus of host MDA-5 signalling pathway Definition: A process in which a symbiont interferes with, inhibits or disrupts a cytoplasmic pattern recognition receptor signaling pathway by inhibiting the activity of MDA-5 (also known as IFIH1). The cytoplasmic pattern recognition receptor MDA-5 detects dsRNA synthesized during active viral replication and triggers a signaling pathway to protect the host against viral infection, for example by inducing the expression of antiviral cytokines. References: PMID:19019954, PMID:33727702